alpha-beta T cell activation [GO:0046631] (BP) Regulation: regulated by regulation of alpha-beta T cell activation [GO:0046634]; positively regulated by positive regulation of alpha-beta T cell activation [GO:0046635]; negatively regulated by GO:0046636 Sources: GOC:add Also known as: alpha-beta T lymphocyte activation, alpha-beta T-cell activation, alpha-beta T-lymphocyte activation Subtypes: alpha-beta T cell activation involved in immune response [GO:0002287], CD4-positive, alpha-beta T cell activation [GO:0035710], CD8-positive, alpha-beta T cell activation [GO:0036037], alpha-beta T cell activation by superantigen [GO:0042722], GO:0046632, GO:0046633, NK T cell activation [GO:0051132] Relationships: is a type of T cell activation [GO:0042110] Definition: The change in morphology and behavior of an alpha-beta T cell resulting from exposure to a mitogen, cytokine, chemokine, cellular ligand, or an antigen for which it is specific.